{
  "gene_name": "Serine_threonine-protein kinase Sgk1",
  "gene_symbol": "SGK1",
  "gene": "UniProtKB:O00141",
  "term_label": "potassium channel regulator activity",
  "term_id": "GO:0015459"
}